{
  "gene": "UniProtKB:Q8IUR5",
  "term_label": "Unknown cellular component",
  "gene_symbol": "TMTC1",
  "term_id": "UNKNOWN:0003",
  "gene_name": "Protein O-mannosyl-transferase TMTC1"
}